mammary gland branching involved in pregnancy [GO:0060745] (biological process) Definition: The process in which the branching structure of the mammary gland duct is generated and organized as a part of pregnancy. Relationships: is a type of developmental process involved in reproduction [GO:0003006]; is a type of maternal process involved in female pregnancy [GO:0060135]; is a type of GO:0060444 References: PMID:19261859 Sources: GOC:dph